sphingosine-1-phosphate phosphatase activity [GO:0042392] (molecular function) Also known as: SPP phosphatase activity, SPPase activity, sphingosine-1-phosphate phosphohydrolase activity Definition: Catalysis of the reaction: sphingosine 1-phosphate + H2O = sphingosine + phosphate. References: PMID:8663293 Sources: GOC:jl Relationships: is a type of GO:0042577